{
  "gene_name": "Pleckstrin homology domain-containing family O member 1",
  "term_id": "GO:0036195",
  "term_label": "muscle cell projection membrane",
  "gene_symbol": "PLEKHO1",
  "gene": "UniProtKB:Q53GL0"
}